{
  "gene_symbol": "SYAP1",
  "gene_name": "Synapse-associated protein 1",
  "term_id": "GO:0005634",
  "term_label": "nucleus",
  "gene": "UniProtKB:Q96A49"
}